{
  "term_label": "Unknown cellular component",
  "gene_name": "Olfactory receptor 4F4",
  "gene": "UniProtKB:Q96R69",
  "term_id": "UNKNOWN:0003",
  "gene_symbol": "OR4F4"
}